{
  "gene_symbol": "SIN3B",
  "term_id": "GO:0000785",
  "gene": "UniProtKB:O75182",
  "gene_name": "Paired amphipathic helix protein Sin3b",
  "term_label": "chromatin"
}